{
  "gene_symbol": "FRMD5",
  "gene_name": "FERM domain-containing protein 5",
  "term_label": "cytoskeleton",
  "gene": "UniProtKB:Q7Z6J6",
  "term_id": "GO:0005856"
}